ribonucleoside monophosphate biosynthetic process [GO:0009156] (biological process) Relationships: is_a GO:0009124 Subtypes: purine ribonucleoside monophosphate biosynthetic process [GO:0009168], pyrimidine ribonucleoside monophosphate biosynthetic process [GO:0009174], FMN biosynthetic process [GO:0009398], GO:0120232 Also known as: ribonucleoside monophosphate anabolism, ribonucleoside monophosphate biosynthesis, ribonucleoside monophosphate formation, ribonucleoside monophosphate synthesis Sources: GOC:go_curators, ISBN:0198506732 Definition: The chemical reactions and pathways resulting in the formation of a ribonucleoside monophosphate, a compound consisting of a nucleobase linked to a ribose sugar esterified with phosphate on the sugar.